{
  "term_id": "GO:0005912",
  "gene": "UniProtKB:Q15124",
  "gene_name": "Phosphoglucomutase-like protein 5",
  "term_label": "adherens junction",
  "gene_symbol": "PGM5"
}